{
  "gene_symbol": "RGL1",
  "gene_name": "Ral guanine nucleotide dissociation stimulator-like 1",
  "term_label": "Ras protein signal transduction",
  "term_id": "GO:0007265",
  "gene": "UniProtKB:Q9NZL6"
}